phospholipid homeostasis [GO:0055091] (biological process) Sources: GOC:BHF, GOC:rl Definition: Any process involved in the maintenance of an internal steady state of phospholipid within an organism or cell. Relationships: is a type of GO:0055088